(S)-N-acetyl-1-phenylethylamine hydrolase activity [GO:0050536] (molecular function) Also known as: (S)-N-acetyl-1-phenylethylamine amidohydrolase activity, (S)-N-acetylphenylethylamine:H2O hydrolase activity Definition: Catalysis of the reaction: N-acetylphenylethylamine + H2O = acetate + phenylethylamine. Sources: EC:3.5.1.85, RHEA:23952 Relationships: is a type of hydrolase activity, acting on carbon-nitrogen (but not peptide) bonds, in linear amides [GO:0016811]